{
  "term_label": "protein transport to vacuole involved in ubiquitin-dependent protein catabolic process via the multivesicular body sorting pathway",
  "term_id": "GO:0043328",
  "gene_name": "Vacuolar protein sorting-associated protein 28 homolog",
  "gene": "UniProtKB:Q9UK41",
  "gene_symbol": "VPS28"
}